{
  "gene_name": "Choline-phosphate cytidylyltransferase B",
  "term_label": "Unknown biological process",
  "gene_symbol": "PCYT1B",
  "term_id": "UNKNOWN:0002",
  "gene": "UniProtKB:Q9Y5K3"
}